{
  "gene_symbol": "TAFA2",
  "term_id": "GO:0048018",
  "gene_name": "Chemokine-like protein TAFA-2",
  "gene": "UniProtKB:Q8N3H0",
  "term_label": "receptor ligand activity"
}